{
  "gene": "UniProtKB:O15438",
  "term_id": "GO:0055085",
  "gene_name": "ATP-binding cassette sub-family C member 3",
  "gene_symbol": "ABCC3",
  "term_label": "transmembrane transport"
}